compound eye photoreceptor development [GO:0042051] (biological process) Subtypes: GO:0045463, R7 cell development [GO:0045467], R1/R6 development [GO:0048053], GO:0048055, R3/R4 development [GO:0048057] Also known as: adult eye photoreceptor development Relationships: is a type of eye photoreceptor cell development [GO:0042462]; is part of compound eye photoreceptor cell differentiation [GO:0001751] Regulation: regulated by regulation of compound eye photoreceptor development [GO:0045314]; positively regulated by GO:0045315; negatively regulated by negative regulation of compound eye photoreceptor development [GO:0045316] Definition: The process whose specific outcome is the progression of a light-responsive receptor in the compound eye over time, from its formation to the mature structure. Sources: GOC:bf